{
  "gene_name": "Cysteine-rich DPF motif domain-containing protein 1",
  "term_id": "UNKNOWN:0002",
  "gene_symbol": "CDPF1",
  "term_label": "Unknown biological process",
  "gene": "UniProtKB:Q6NVV7"
}